phenol-containing compound biosynthetic process [GO:0046189] (biological process) Subtypes: octopamine biosynthetic process [GO:0006589], salicylic acid biosynthetic process [GO:0009697], GO:0009713, proanthocyanidin biosynthetic process [GO:0010023], DIF-1 biosynthetic process [GO:0031148], GO:0033495, sinapate biosynthetic process [GO:0033497], sinapate ester biosynthetic process [GO:0033525], asperthecin biosynthetic process [GO:0036184], GO:0042189, GO:0042427, melanin biosynthetic process [GO:0042438], eugenol biosynthetic process [GO:0042855], pyochelin biosynthetic process [GO:0042864], novobiocin biosynthetic process [GO:0043642], aerobic phenol-containing compound biosynthetic process [GO:0046190], anaerobic phenol-containing compound biosynthetic process [GO:0046192], orcinol biosynthetic process [GO:0046197], cichorine biosynthetic process [GO:0062032], phenolic phthiocerol biosynthetic process [GO:0097041], zearalenone biosynthetic process [GO:0106150], mycophenolic acid biosynthetic process [GO:0140722], ilicicolin H biosynthetic process [GO:0140781], (M)-viriditoxin biosynthetic process [GO:0140783], viridicatumtoxin biosynthetic process [GO:0140872], diorcinol biosynthetic process [GO:1900572], emodin biosynthetic process [GO:1900575], GO:1900584, GO:1900602, GO:1900611, F-9775B biosynthetic process [GO:1900614], averantin biosynthetic process [GO:1900763], GO:1900766, fonsecin biosynthetic process [GO:1900769], shamixanthone biosynthetic process [GO:1900793], monodictyphenone biosynthetic process [GO:1900815], GO:1901024, GO:1901366, GO:1901599, tyramine biosynthetic process [GO:1901695], olivetolic acid biosynthetic process [GO:1901697], GO:1901786, GO:1901887, neosartoricin biosynthetic process [GO:1902050], GO:1902126, (-)-lariciresinol biosynthetic process [GO:1902129], (+)-lariciresinol biosynthetic process [GO:1902132], (+)-secoisolariciresinol biosynthetic process [GO:1902135], (-)-secoisolariciresinol biosynthetic process [GO:1902138] Also known as: phenol-containing compound anabolism, phenol-containing compound biosynthesis, phenol-containing compound formation, phenol-containing compound synthesis Relationships: is a type of biosynthetic process [GO:0009058]; is a type of GO:0018958 Definition: The chemical reactions and pathways resulting in the formation of a phenol, any compound containing one or more hydroxyl groups directly attached to an aromatic carbon ring. Sources: GOC:ai